{
  "gene_symbol": "C6orf226",
  "gene_name": "Uncharacterized protein C6orf226",
  "term_label": "Unknown biological process",
  "gene": "UniProtKB:Q5I0X4",
  "term_id": "UNKNOWN:0002"
}